{
  "gene_symbol": "LAT2",
  "gene": "UniProtKB:Q9GZY6",
  "gene_name": "Linker for activation of T-cells family member 2",
  "term_label": "Unknown molecular function",
  "term_id": "UNKNOWN:0001"
}